{
  "gene_name": "Putative golgin subfamily A member 2B",
  "term_id": "UNKNOWN:0003",
  "gene_symbol": "GOLGA2P5",
  "term_label": "Unknown cellular component",
  "gene": "UniProtKB:Q9HBQ8"
}